negative regulation of imaginal disc-derived leg joint morphogenesis [GO:0110139] (biological process) Relationships: is a type of negative regulation of developmental process [GO:0051093]; is a type of regulation of imaginal disc-derived leg joint morphogenesis [GO:0110137]; negatively regulates imaginal disc-derived leg morphogenesis [GO:0007480] References: PMID:25329825 Sources: GOC:ha Definition: Any process that stops, prevents, or reduces the frequency, rate or extent of imaginal disc-derived leg joint morphogenesis.